cytoplasmic translational elongation [GO:0002182] (BP) Definition: The successive addition of amino acid residues to a nascent polypeptide chain during protein biosynthesis in the cytoplasm. Relationships: is a type of translational elongation [GO:0006414]; is part of cytoplasmic translation [GO:0002181] Sources: GOC:hjd Regulation: regulated by regulation of cytoplasmic translational elongation [GO:1900247]; negatively regulated by negative regulation of cytoplasmic translational elongation [GO:1900248]; positively regulated by GO:1900249 Subtypes: cytoplasmic translational elongation through polyproline stretches [GO:0097622], CAT tailing [GO:0140708]